{
  "term_id": "UNKNOWN:0002",
  "term_label": "Unknown biological process",
  "gene": "UniProtKB:Q9H190",
  "gene_name": "Syntenin-2",
  "gene_symbol": "SDCBP2"
}